{
  "term_label": "Unknown molecular function",
  "term_id": "UNKNOWN:0001",
  "gene_name": "CEP295 N-terminal-like protein",
  "gene_symbol": "CEP295NL",
  "gene": "UniProtKB:Q96MC4"
}